{
  "term_id": "GO:0004888",
  "term_label": "transmembrane signaling receptor activity",
  "gene_name": "Neurexin-3",
  "gene_symbol": "NRXN3",
  "gene": "UniProtKB:Q9Y4C0"
}